{
  "gene_name": "Calpain-14",
  "gene": "UniProtKB:A8MX76",
  "gene_symbol": "CAPN14",
  "term_label": "proteolysis",
  "term_id": "GO:0006508"
}